{
  "term_id": "UNKNOWN:0001",
  "term_label": "Unknown molecular function",
  "gene": "UniProtKB:Q5VV43",
  "gene_symbol": "KIAA0319",
  "gene_name": "Dyslexia-associated protein KIAA0319"
}